{
  "gene": "UniProtKB:O14933",
  "gene_name": "Ubiquitin_ISG15-conjugating enzyme E2 L6",
  "gene_symbol": "UBE2L6",
  "term_id": "GO:0042296",
  "term_label": "ISG15 transferase activity"
}